{
  "term_label": "chloride transmembrane transport",
  "gene_name": "Gamma-aminobutyric acid receptor subunit alpha-5",
  "gene_symbol": "GABRA5",
  "gene": "UniProtKB:P31644",
  "term_id": "GO:1902476"
}